{
  "gene_symbol": "PAGE5",
  "term_label": "Unknown biological process",
  "term_id": "UNKNOWN:0002",
  "gene_name": "P antigen family member 5",
  "gene": "UniProtKB:Q96GU1"
}